{
  "gene_name": "Protocadherin alpha-10",
  "term_label": "cell adhesion molecule binding",
  "gene": "UniProtKB:Q9Y5I2",
  "term_id": "GO:0050839",
  "gene_symbol": "PCDHA10"
}